{
  "term_id": "GO:0016018",
  "gene_symbol": "PPIAL4A",
  "gene_name": "Peptidyl-prolyl cis-trans isomerase A-like 4A",
  "gene": "UniProtKB:Q9Y536",
  "term_label": "cyclosporin A binding"
}